regulation of Rac protein signal transduction [GO:0035020] (biological process) Subtypes: negative regulation of Rac protein signal transduction [GO:0035021], positive regulation of Rac protein signal transduction [GO:0035022] Relationships: is_a GO:0051056; regulates Rac protein signal transduction [GO:0016601] Definition: Any process that modulates the frequency, rate or extent of Rac protein signal transduction. Sources: GOC:bf